symbiont-mediated suppression of host ISG15-protein conjugation [GO:0039579] (biological process) Also known as: suppression by virus of host ISG15-protein conjugation, suppression by virus of host ISG15 activity References: PMID:11157743, PMID:18078692, PMID:18604270, PMID:32845033 Relationships: is a type of symbiont-mediated suppression of host innate immune response [GO:0052170] Definition: Any process in which a symbiont inhibits or disrupts a host ubiquitin-like protein ISG15 conjugation to a substrate. ISG15 is a ubiquitin-like protein that is conjugated to lysine residues on various target proteins. For example, some viruses escape the antiviral activity of ISG15 by using different mechanisms; the influenza B virus NS1 protein blocks the covalent linkage of ISG15 to its target proteins by directly interacting with ISG15, while the papain-like protease from the coronavirus cleaves ISG15 derivatives.